cholinesterase activity [GO:0004104] (molecular function) Definition: Catalysis of the reaction: an acylcholine + H2O = choline + a carboxylic acid anion. Relationships: is_a GO:0052689 Subtypes: GO:0003990 Also known as: BtChoEase activity, acylcholine acylhydrolase activity, anticholineesterase activity, benzoylcholinesterase activity, butyrylcholine esterase activity, butyrylcholinesterase activity, choline esterase II (unspecific) activity, choline esterase activity, non-specific cholinesterase activity, propionylcholinesterase activity, pseudocholinesterase activity Sources: EC:3.1.1.8